{
  "gene_symbol": "ZNF432",
  "term_id": "UNKNOWN:0003",
  "gene_name": "Zinc finger protein 432",
  "gene": "UniProtKB:O94892",
  "term_label": "Unknown cellular component"
}